{
  "gene_name": "Uncharacterized protein",
  "term_label": "Unknown molecular function",
  "term_id": "UNKNOWN:0001",
  "gene": "UniProtKB:A0A1W2PNU3",
  "gene_symbol": "LOC122455342"
}